{
  "gene_name": "Ret finger protein-like 4B",
  "term_id": "GO:0005737",
  "term_label": "cytoplasm",
  "gene": "UniProtKB:Q6ZWI9",
  "gene_symbol": "RFPL4B"
}